positive regulation of heart growth [GO:0060421] (biological process) Definition: Any process that increases the rate or extent of heart growth. Heart growth is the increase in size or mass of the heart. Sources: GOC:BHF, GOC:dph, GOC:tb Relationships: is_a positive regulation of organ growth [GO:0046622]; is a type of GO:0060420; positively regulates heart growth [GO:0060419] Subtypes: positive regulation of cardiac muscle tissue growth [GO:0055023]